{
  "gene": "UniProtKB:P17022",
  "gene_symbol": "ZNF18",
  "term_label": "RNA polymerase II cis-regulatory region sequence-specific DNA binding",
  "gene_name": "Zinc finger protein 18",
  "term_id": "GO:0000978"
}